response to fluoride [GO:1902617] (biological process) References: PMID:8138152 Sources: GOC:TermGenie, GOC:kmv, GO_REF:0000071 Subtypes: cellular response to fluoride [GO:1902618] Relationships: is_a GO:0042221 Definition: Any process that results in a change in state or activity of a cell or an organism (in terms of movement, secretion, enzyme production, gene expression, etc.) as a result of a fluoride stimulus.